suckling behavior [GO:0001967] (biological process) Definition: Specific behavior of a newborn or infant mammal that results in the derivation of nourishment from the breast. Sources: GOC:dph, GOC:pr Also known as: nursing behavior Relationships: is a type of GO:0007631